{
  "gene_symbol": "TRAJ19",
  "gene_name": "T cell receptor alpha joining 19 (non-functional) (Fragment)",
  "gene": "UniProtKB:A0A075B6Y4",
  "term_label": "Unknown molecular function",
  "term_id": "UNKNOWN:0001"
}